hydroxypyruvate decarboxylase activity [GO:0047997] (molecular function) Definition: Catalysis of the reaction: 3-hydroxypyruvate + H+ = CO2 + glycolaldehyde. Sources: EC:4.1.1.40, RHEA:20561 Also known as: hydroxypyruvate carboxy-lyase (glycolaldehyde-forming), hydroxypyruvate carboxy-lyase activity Relationships: is a type of carboxy-lyase activity [GO:0016831]